{
  "gene_name": "Peroxisomal acyl-coenzyme A oxidase 1",
  "term_label": "peroxisome",
  "gene_symbol": "ACOX1",
  "term_id": "GO:0005777",
  "gene": "UniProtKB:Q15067"
}